{
  "term_id": "UNKNOWN:0002",
  "gene_symbol": "C8orf89",
  "gene": "UniProtKB:P0DMQ9",
  "term_label": "Unknown biological process",
  "gene_name": "Putative uncharacterized protein C8orf89"
}